{
  "gene": "UniProtKB:Q8TC20",
  "term_id": "UNKNOWN:0002",
  "term_label": "Unknown biological process",
  "gene_symbol": "CAGE1",
  "gene_name": "Cancer-associated gene 1 protein"
}